{
  "term_id": "GO:0070213",
  "term_label": "protein auto-ADP-ribosylation",
  "gene_name": "Protein mono-ADP-ribosyltransferase PARP11",
  "gene": "UniProtKB:Q9NR21",
  "gene_symbol": "PARP11"
}